malic enzyme activity [GO:0004470] (molecular function) Subtypes: GO:0004471, malate dehydrogenase (decarboxylating) (NADP+) activity [GO:0004473] Sources: ISBN:0198506732 Also known as: pyruvic-malic carboxylase activity Definition: Catalysis of the oxidative decarboxylation of malate with the concomitant production of pyruvate. Relationships: is_a malate dehydrogenase activity [GO:0016615]